{
  "gene_symbol": "JRK",
  "gene": "UniProtKB:O75564",
  "term_label": "Unknown biological process",
  "term_id": "UNKNOWN:0002",
  "gene_name": "Jerky protein homolog"
}